insulin-responsive D-glucose:proton symporter activity [GO:0005360] (molecular function) Also known as: insulin-responsive glucose:proton symporter activity, insulin-responsive hydrogen:glucose symporter activity, insulin-responsive hydrogen:glucose transporter activity, transepithelial hydrogen/glucose transporter activity Sources: GOC:mtg_transport Relationships: is_a GO:0005356 Definition: Enables the transfer of a solute or solutes from one side of a membrane to the other according to the reaction: glucose(out) + H(out)+ = glucose(in) + H(in)+, in response to a stimulus by insulin. Symporter activity enables the active transport of a solute across a membrane by a mechanism whereby two or more species are transported together in the same direction in a tightly coupled process not directly linked to a form of energy other than chemiosmotic energy.